{
  "gene_symbol": "CR1L",
  "term_id": "GO:0002456",
  "gene_name": "Complement component receptor 1-like protein",
  "term_label": "T cell mediated immunity",
  "gene": "UniProtKB:Q2VPA4"
}